{
  "gene_symbol": "NPY6R",
  "gene_name": "Putative neuropeptide Y receptor type 6",
  "gene": "UniProtKB:Q99463",
  "term_id": "UNKNOWN:0002",
  "term_label": "Unknown biological process"
}